{
  "gene_name": "Zinc finger protein 649",
  "gene": "UniProtKB:Q9BS31",
  "term_label": "regulation of transcription by RNA polymerase II",
  "term_id": "GO:0006357",
  "gene_symbol": "ZNF649"
}